{
  "gene": "UniProtKB:O15050",
  "gene_symbol": "TRANK1",
  "term_id": "UNKNOWN:0003",
  "term_label": "Unknown cellular component",
  "gene_name": "TPR and ankyrin repeat-containing protein 1"
}